DNA strand elongation involved in cell cycle DNA replication [GO:1902296] (biological process) Sources: GOC:TermGenie, GOC:mtg_cell_cycle Also known as: DNA replication elongation involved in cell cycle DNA replication, DNA strand elongation during DNA replication involved in cell cycle DNA replication Relationships: is a type of DNA strand elongation involved in DNA replication [GO:0006271]; is a type of cell cycle process [GO:0022402]; is part of cell cycle DNA replication [GO:0044786] Subtypes: DNA strand elongation involved in nuclear cell cycle DNA replication [GO:1902319] Definition: Any DNA strand elongation that is involved in cell cycle DNA replication.